{
  "gene": "UniProtKB:Q9HB40",
  "term_label": "Unknown biological process",
  "gene_symbol": "SCPEP1",
  "gene_name": "Retinoid-inducible serine carboxypeptidase",
  "term_id": "UNKNOWN:0002"
}